{
  "term_label": "plasma membrane",
  "term_id": "GO:0005886",
  "gene_symbol": "MICAL1",
  "gene_name": "[F-actin]-monooxygenase MICAL1",
  "gene": "UniProtKB:Q8TDZ2"
}